{
  "term_label": "S100 protein binding",
  "gene": "UniProtKB:P23297",
  "gene_name": "Protein S100-A1",
  "term_id": "GO:0044548",
  "gene_symbol": "S100A1"
}